cholesterol biosynthetic process via lathosterol [GO:0033490] (biological process) Also known as: cholesterol anabolism via lathosterol, cholesterol biosynthesis via lathosterol, cholesterol formation via lathosterol, cholesterol synthesis via lathosterol Definition: The chemical reactions and pathways resulting in the formation of cholesterol, cholest-5-en-3 beta-ol, via the intermediate lathosterol. Relationships: is a type of cholesterol biosynthetic process [GO:0006695] Sources: GOC:mah, MetaCyc:PWY66-341